{
  "term_id": "GO:0046856",
  "term_label": "phosphatidylinositol dephosphorylation",
  "gene_name": "Myotubularin-related protein 4",
  "gene": "UniProtKB:Q9NYA4",
  "gene_symbol": "MTMR4"
}